{
  "term_label": "olfactory receptor activity",
  "gene": "UniProtKB:Q6IEZ7",
  "gene_symbol": "OR2T5",
  "term_id": "GO:0004984",
  "gene_name": "Olfactory receptor 2T5"
}